L-methionine catabolic process to 3-methylthiopropanol [GO:0000951] (BP) Relationships: is a type of amino acid catabolic process to alcohol via Ehrlich pathway [GO:0000947]; is a type of L-methionine catabolic process [GO:0009087]; is a type of sulfur compound biosynthetic process [GO:0044272] Definition: The chemical reactions and pathways involving the catabolism of branched chain amino acids to produce branched chain alcohols with one carbon less than the starting amino acid. In S. cerevisiae, this is known to occur for leucine, isoleucine, valine, methionine, phenylalanine, tyrosine, or tryptophan. When L-methionine is used as the substrate, 3-methylthiopropanol is produced. Often referred to as the Ehrlich pathway, these reactions generally occur during fermentation to produce a variety of alcohols, often collectively referred to as fusel alcohols. Depending on the redox state of the cells, carboxylic acid derivatives may be produced instead of alcohols. References: PMID:18281432 Sources: GOC:krc